protein localization to division septum [GO:1902432] (biological process) Definition: A process in which a protein is transported to, or maintained in, a location within a division septum. References: PMID:9367977 Sources: GOC:TermGenie Relationships: is a type of protein localization to cell division site [GO:0072741] Also known as: protein localisation in division septum, protein localisation to division septum, protein localization in division septum